{
  "gene": "UniProtKB:Q8NE35",
  "gene_symbol": "CPEB3",
  "term_id": "GO:0003730",
  "term_label": "mRNA 3'-UTR binding",
  "gene_name": "Cytoplasmic polyadenylation element-binding protein 3"
}